{
  "gene_symbol": "FGFR3",
  "term_id": "GO:0017134",
  "term_label": "fibroblast growth factor binding",
  "gene": "UniProtKB:P22607",
  "gene_name": "Fibroblast growth factor receptor 3"
}